{
  "gene": "UniProtKB:P61927",
  "gene_name": "Large ribosomal subunit protein eL37",
  "term_id": "GO:0022625",
  "gene_symbol": "RPL37",
  "term_label": "cytosolic large ribosomal subunit"
}